{
  "term_label": "vesicle docking involved in exocytosis",
  "gene_symbol": "STXBP2",
  "gene": "UniProtKB:Q15833",
  "term_id": "GO:0006904",
  "gene_name": "Syntaxin-binding protein 2"
}